{
  "gene": "UniProtKB:O75038",
  "gene_symbol": "PLCH2",
  "gene_name": "1-phosphatidylinositol 4,5-bisphosphate phosphodiesterase eta-2",
  "term_label": "Unknown cellular component",
  "term_id": "UNKNOWN:0003"
}